{
  "gene_symbol": "HOXC12",
  "term_label": "Unknown biological process",
  "gene_name": "Homeobox protein Hox-C12",
  "gene": "UniProtKB:P31275",
  "term_id": "UNKNOWN:0002"
}